ERBB3 signaling pathway [GO:0038129] (biological process) Subtypes: ERBB2-ERBB3 signaling pathway [GO:0038133], ERBB3-ERBB4 signaling pathway [GO:0038136] Regulation: regulated by GO:1905578; RO_0002212 by negative regulation of ERBB3 signaling pathway [GO:1905579]; positively regulated by positive regulation of ERBB3 signaling pathway [GO:1905580] Definition: The series of molecular signals initiated by binding of a ligand to the tyrosine kinase receptor ERBB3 on the surface of a cell, and ending with the regulation of a downstream cellular process, e.g. transcription. ERBB3 receptors have impaired kinase activity and rely on the kinase activity of the heterodimer partner for activation and signal transmission. References: PMID:16460914 Sources: GOC:jc Also known as: ERBB3 signalling pathway, HER3 signaling pathway, receptor tyrosine-protein kinase erbB-3 signaling pathway Relationships: is a type of ERBB signaling pathway [GO:0038127]